{
  "term_label": "negative regulation of transcription by RNA polymerase II",
  "term_id": "GO:0000122",
  "gene_symbol": "HIC2",
  "gene": "UniProtKB:Q96JB3",
  "gene_name": "Hypermethylated in cancer 2 protein"
}